{
  "term_id": "GO:0000493",
  "gene_name": "H_ACA ribonucleoprotein complex non-core subunit NAF1",
  "term_label": "box H/ACA snoRNP assembly",
  "gene": "UniProtKB:Q96HR8",
  "gene_symbol": "NAF1"
}